{
  "gene": "UniProtKB:P09769",
  "gene_name": "Tyrosine-protein kinase Fgr",
  "term_id": "GO:0007229",
  "term_label": "integrin-mediated signaling pathway",
  "gene_symbol": "FGR"
}